all-trans-retinol dehydrogenase (NADP+) activity [GO:0052650] (molecular function) Also known as: all-trans retinal reductase activity, all-trans-retinol dehydrogenase activity, retinol dehydrogenase activity, NADP-retinol dehydrogenase activity, NADP(H)-dependent retinol dehydrogenase/reductase activity, retinol dehydrogenase [NADP+] activity, retinol:NADP+ oxidoreductase activity Definition: Catalysis of the reaction: all-trans-retinol + NADP+ = all-trans-retinal + NADPH + H+. Relationships: is a type of alcohol dehydrogenase (NADP+) activity [GO:0008106]; BFO_0000050 retinol metabolic process [GO:0042572] Sources: RHEA:25033